{
  "term_label": "anterograde synaptic vesicle transport",
  "gene": "UniProtKB:Q13367",
  "gene_symbol": "AP3B2",
  "gene_name": "AP-3 complex subunit beta-2",
  "term_id": "GO:0048490"
}